{
  "gene": "UniProtKB:Q7Z2W4",
  "term_id": "GO:0009615",
  "gene_name": "Zinc finger CCCH-type antiviral protein 1",
  "gene_symbol": "ZC3HAV1",
  "term_label": "response to virus"
}